negative regulation of cardiac chamber formation [GO:1901211] (biological process) Definition: Any process that stops, prevents or reduces the frequency, rate or extent of cardiac chamber formation. Relationships: is_a negative regulation of developmental process [GO:0051093]; is a type of regulation of cardiac chamber formation [GO:1901210]; negatively regulates cardiac chamber formation [GO:0003207] Subtypes: negative regulation of cardiac ventricle formation [GO:1904943] Sources: GOC:BHF, GOC:TermGenie Also known as: down regulation of cardiac chamber formation, down regulation of heart chamber formation, down-regulation of cardiac chamber formation, down-regulation of heart chamber formation, downregulation of cardiac chamber formation, downregulation of heart chamber formation, inhibition of heart chamber formation, negative regulation of heart chamber formation, inhibition of cardiac chamber formation